{
  "gene": "UniProtKB:O95456",
  "term_id": "GO:0080129",
  "gene_symbol": "PSMG1",
  "gene_name": "Proteasome assembly chaperone 1",
  "term_label": "proteasome core complex assembly"
}